{
  "gene": "UniProtKB:O14662",
  "term_label": "endomembrane system",
  "gene_name": "Syntaxin-16",
  "term_id": "GO:0012505",
  "gene_symbol": "STX16"
}